superior olivary nucleus structural organization [GO:0021721] (biological process) Sources: GOC:cls, GOC:dgh, GOC:dph, GOC:jid, GO_REF:0000021 Also known as: superior olivary nucleus structural organisation Relationships: is a type of anatomical structure arrangement [GO:0048532]; is part of GO:0021585; is part of superior olivary nucleus morphogenesis [GO:0021719] Definition: The process that contributes to the act of creating the structural organization of the superior olivary nucleus structure. In mice, the superior olivary nucleus is a small cylindrical mass on the dorsal surface of the lateral part of the trapezoid body of the pons, and it is situated immediately above the inferior olivary nucleus. It receives projections from the cochlear nucleus and thus is involved in the perception of sound.